{
  "term_id": "UNKNOWN:0001",
  "gene_name": "T cell receptor beta joining 2-4",
  "gene": "UniProtKB:A0A0A0MT87",
  "gene_symbol": "TRBJ2-4",
  "term_label": "Unknown molecular function"
}